{
  "gene_symbol": "GTF3A",
  "gene_name": "Transcription factor IIIA",
  "term_id": "UNKNOWN:0001",
  "term_label": "Unknown molecular function",
  "gene": "UniProtKB:Q92664"
}